negative regulation of chronic inflammatory response to antigenic stimulus [GO:0002875] (biological process) Relationships: is a type of negative regulation of chronic inflammatory response [GO:0002677]; is a type of negative regulation of inflammatory response to antigenic stimulus [GO:0002862]; is a type of regulation of chronic inflammatory response to antigenic stimulus [GO:0002874]; negatively regulates chronic inflammatory response to antigenic stimulus [GO:0002439] Sources: GOC:add Also known as: down regulation of chronic inflammatory response to antigenic stimulus, down-regulation of chronic inflammatory response to antigenic stimulus, downregulation of chronic inflammatory response to antigenic stimulus, inhibition of chronic inflammatory response to antigenic stimulus Definition: Any process that stops, prevents, or reduces the frequency, rate, or extent of a chronic inflammatory response to an antigenic stimulus.